femoral head articular cartilage development [GO:0061979] (biological process) Definition: The process whose specific outcome is the progression of femoral head articular cartilage over time, from its formation to the mature structure. Relationships: is a type of GO:0061977 References: PMID:20097540